{
  "term_id": "GO:0042803",
  "gene_name": "Teneurin-3",
  "term_label": "protein homodimerization activity",
  "gene_symbol": "TENM3",
  "gene": "UniProtKB:Q9P273"
}